{
  "term_id": "GO:0005525",
  "gene": "UniProtKB:P23258",
  "gene_name": "Tubulin gamma-1 chain",
  "gene_symbol": "TUBG1",
  "term_label": "GTP binding"
}